{
  "term_id": "UNKNOWN:0001",
  "gene": "UniProtKB:Q9ULZ1",
  "term_label": "Unknown molecular function",
  "gene_symbol": "APLN",
  "gene_name": "Apelin"
}